fumitremorgin B biosynthetic process [GO:1900772] (biological process) Relationships: is a type of indole alkaloid biosynthetic process [GO:0035835] References: PMID:18683158 Sources: GOC:TermGenie, GOC:di Also known as: fumitremorgin B metabolic process, fumitremorgin B anabolism, fumitremorgin B biosynthesis, fumitremorgin B formation, fumitremorgin B metabolism, fumitremorgin B synthesis, Lanosulin anabolism, Lanosulin biosynthesis, Lanosulin biosynthetic process, Lanosulin formation, Lanosulin metabolic process, Lanosulin metabolism, Lanosulin synthesis Definition: The chemical reactions and pathways resulting in the formation of the indole alkaloid fumitremorgin B.